Hsp70 protein binding [GO:0030544] (molecular function) Definition: Binding to a Hsp70 protein, heat shock proteins around 70kDa in size. Relationships: is a type of heat shock protein binding [GO:0031072]; is a type of protein-folding chaperone binding [GO:0051087] Sources: ISBN:0198506732